{
  "term_label": "extracellular matrix structural constituent",
  "gene": "UniProtKB:P98095",
  "term_id": "GO:0005201",
  "gene_name": "Fibulin-2",
  "gene_symbol": "FBLN2"
}